regulation of sulfur metabolic process [GO:0042762] (biological process) Definition: Any process that modulates the frequency, rate or extent of the chemical reactions and pathways involving sulfur, the nonmetallic element sulfur or compounds that contain sulfur. Sources: GOC:go_curators Also known as: regulation of sulfur metabolism, regulation of sulphur metabolic process, regulation of sulphur metabolism Relationships: is a type of regulation of metabolic process [GO:0019222]; regulates sulfur compound metabolic process [GO:0006790] Subtypes: regulation of glucosinolate biosynthetic process [GO:0010439], positive regulation of penicillin metabolic process [GO:0033246], regulation of penicillin catabolic process [GO:0033247], regulation of acyl-CoA biosynthetic process [GO:0050812], regulation of taurine biosynthetic process [GO:0062089], GO:0070616, regulation of thiamine biosynthetic process [GO:0070623], GO:0080020, GO:1900058, GO:1900196, regulation of methane biosynthetic process from 3-(methylthio)propionic acid [GO:1900333], regulation of methane biosynthetic process from dimethyl sulfide [GO:1900342], GO:1900345, regulation of butyryl-CoA catabolic process to butanol [GO:1900497], GO:1900500, GO:1900689, GO:1901183, regulation of tetrapyrrole biosynthetic process from glycine and succinyl-CoA [GO:1901413], regulation of cysteine metabolic process [GO:1901494], regulation of glutathione biosynthetic process [GO:1903786], regulation of hydrogen sulfide biosynthetic process [GO:1904826], GO:1905722, GO:2001210